{
  "term_label": "manchette",
  "term_id": "GO:0002177",
  "gene": "UniProtKB:A6NJZ7",
  "gene_symbol": "RIMBP3C",
  "gene_name": "RIMS-binding protein 3C"
}